{
  "gene": "UniProtKB:P0C7X1",
  "term_label": "GTPase activator activity",
  "gene_symbol": "TBC1D3H",
  "gene_name": "TBC1 domain family member 3H",
  "term_id": "GO:0005096"
}